negative regulation of lipid transport [GO:0032369] (biological process) Subtypes: negative regulation of sterol transport [GO:0032372], negative regulation of intracellular lipid transport [GO:0032378], GO:0045972, negative regulation of acylglycerol transport [GO:1901507], negative regulation of lipid transport across blood-brain barrier [GO:1903001], negative regulation of fatty acid transport [GO:2000192], negative regulation of steroid hormone secretion [GO:2000832], GO:2000838, negative regulation of dehydroepiandrosterone secretion [GO:2000841], GO:2000844, negative regulation of phospholipid transport [GO:2001139] Also known as: down regulation of lipid transport, down-regulation of lipid transport, downregulation of lipid transport, inhibition of lipid transport Definition: Any process that stops, prevents, or reduces the frequency, rate or extent of the directed movement of lipids into, out of or within a cell, or between cells, by means of some agent such as a transporter or pore. Relationships: is a type of regulation of lipid transport [GO:0032368]; is a type of negative regulation of transport [GO:0051051]; is_a negative regulation of lipid localization [GO:1905953]; negatively regulates lipid transport [GO:0006869] Sources: GOC:mah